{
  "term_id": "GO:0045109",
  "gene_name": "Keratin, type II cytoskeletal 71",
  "gene_symbol": "KRT71",
  "gene": "UniProtKB:Q3SY84",
  "term_label": "intermediate filament organization"
}